{
  "term_id": "UNKNOWN:0002",
  "gene_symbol": "NT5DC3",
  "term_label": "Unknown biological process",
  "gene": "UniProtKB:Q86UY8",
  "gene_name": "5'-nucleotidase domain-containing protein 3"
}